{
  "term_label": "fructose 1,6-bisphosphate 1-phosphatase activity",
  "gene_symbol": "FBP2",
  "gene": "UniProtKB:O00757",
  "gene_name": "Fructose-1,6-bisphosphatase isozyme 2",
  "term_id": "GO:0042132"
}